{
  "gene": "UniProtKB:Q96BN8",
  "gene_name": "Ubiquitin thioesterase otulin",
  "term_label": "cysteine-type deubiquitinase activity",
  "gene_symbol": "OTULIN",
  "term_id": "GO:0004843"
}